{
  "gene_symbol": "PSMD1",
  "gene": "UniProtKB:Q99460",
  "term_id": "GO:0034515",
  "term_label": "proteasome storage granule",
  "gene_name": "26S proteasome non-ATPase regulatory subunit 1"
}